regulation of mast cell chemotaxis [GO:0060753] (biological process) Definition: Any process that modulates the rate, frequency or extent of mast cell chemotaxis. Mast cell chemotaxis is the movement of a mast cell in response to an external stimulus. Subtypes: positive regulation of mast cell chemotaxis [GO:0060754], negative regulation of mast cell chemotaxis [GO:0060755] Relationships: is a type of GO:0002688; RO_0002211 mast cell chemotaxis [GO:0002551] Sources: GOC:dph, GOC:tb